imaginal disc fusion [GO:0046528] (biological process) Definition: The process following disc eversion whereby imaginal discs fuse with adjacent disc derivatives to form a continuous adult epidermis. References: PMID:11494317 Relationships: is a type of GO:0009886; is part of GO:0007560